{
  "term_id": "GO:0005829",
  "gene_symbol": "LTA4H",
  "gene": "UniProtKB:P09960",
  "gene_name": "Leukotriene A-4 hydrolase",
  "term_label": "cytosol"
}